negative regulation of cilium-dependent cell motility [GO:1902020] (BP) Definition: Any process that stops, prevents or reduces the frequency, rate or extent of cilium-dependent cell motility. Sources: GOC:TermGenie, GOC:cilia, GOC:jl Also known as: down regulation of ciliary cell motility, down-regulation of ciliary cell motility, downregulation of ciliary cell motility, negative regulation of cilium cell motility, inhibition of ciliary cell motility, negative regulation of ciliary cell motility Relationships: is a type of GO:1902019; is a type of negative regulation of cell motility [GO:2000146]; negatively regulates cilium-dependent cell motility [GO:0060285] Subtypes: negative regulation of flagellated sperm motility [GO:1901318]